{
  "term_label": "protein-macromolecule adaptor activity",
  "gene_symbol": "ERG28",
  "term_id": "GO:0030674",
  "gene": "UniProtKB:Q9UKR5",
  "gene_name": "Ergosterol biosynthetic protein 28 homolog"
}